DNA (6-4) photolyase activity [GO:0003914] (molecular function) Definition: Catalysis of the reaction: pyrimidine-pyrimidone (6-4) photoproduct (in DNA) = 2 pyrimidine residues (in DNA). Catalyzes the reactivation of ultraviolet-irradiated DNA. References: PMID:11124949 Sources: GOC:mah Relationships: is a type of DNA photolyase activity [GO:0003913]